cellular response to formaldehyde [GO:1904405] (biological process) Definition: Any process that results in a change in state or activity of a cell (in terms of movement, secretion, enzyme production, gene expression, etc.) as a result of a formaldehyde stimulus. References: PMID:9149109 Sources: GOC:TermGenie, GO_REF:0000071 Relationships: is a type of cellular response to aldehyde [GO:0110096]; is a type of response to formaldehyde [GO:1904404]